{
  "gene_symbol": "FAM241A",
  "gene": "UniProtKB:Q8N8J7",
  "term_label": "Unknown molecular function",
  "gene_name": "Uncharacterized protein FAM241A",
  "term_id": "UNKNOWN:0001"
}